{
  "gene_symbol": "PMPCA",
  "gene_name": "Mitochondrial-processing peptidase subunit alpha",
  "gene": "UniProtKB:Q10713",
  "term_label": "mitochondrial processing peptidase complex",
  "term_id": "GO:0017087"
}